{
  "gene_name": "Histone deacetylase 7",
  "term_label": "histone deacetylase activity",
  "gene_symbol": "HDAC7",
  "term_id": "GO:0004407",
  "gene": "UniProtKB:Q8WUI4"
}